4-carboxy-4'-sulfoazobenzene metabolic process [GO:0018887] (biological process) References: PMID:9603860 Also known as: 4-carboxy-4'-sulfoazobenzene metabolism, 4-carboxy-4'-sulphoazobenzene metabolic process, 4-carboxy-4'-sulphoazobenzene metabolism Definition: The chemical reactions and pathways involving 4-carboxy-4'-sulfoazobenzene, a sulfonated azo compound synthesized by nitro-amine condensation from sulfanilic acid and 4-nitrobenzoic acid. Relationships: is a type of sulfur compound metabolic process [GO:0006790]; is_a monocarboxylic acid metabolic process [GO:0032787]; is_a benzene-containing compound metabolic process [GO:0042537]